cellular response to rotenone [GO:1904648] (biological process) Definition: Any process that results in a change in state or activity of a cell (in terms of movement, secretion, enzyme production, gene expression, etc.) as a result of a rotenone stimulus. References: PMID:18538940 Sources: GOC:TermGenie, GO_REF:0000071 Relationships: is a type of cellular response to ketone [GO:1901655]; is a type of GO:1904647